{
  "gene": "UniProtKB:Q8TB36",
  "gene_symbol": "GDAP1",
  "term_label": "mitochondrial fusion",
  "term_id": "GO:0008053",
  "gene_name": "Ganglioside-induced differentiation-associated protein 1"
}